{
  "gene_symbol": "CEP295",
  "gene": "UniProtKB:Q9C0D2",
  "term_label": "regulation of centriole replication",
  "term_id": "GO:0046599",
  "gene_name": "Centrosomal protein of 295 kDa"
}